{
  "gene_name": "AT-rich interactive domain-containing protein 1B",
  "term_label": "regulation of transcription by RNA polymerase II",
  "gene": "UniProtKB:Q8NFD5",
  "term_id": "GO:0006357",
  "gene_symbol": "ARID1B"
}